{
  "term_id": "GO:0072583",
  "term_label": "clathrin-dependent endocytosis",
  "gene_symbol": "FCHO2",
  "gene_name": "F-BAR domain only protein 2",
  "gene": "UniProtKB:Q0JRZ9"
}